{
  "gene_symbol": "PHAF1",
  "gene_name": "Phagosome assembly factor 1",
  "gene": "UniProtKB:Q9BSU1",
  "term_id": "GO:0005802",
  "term_label": "trans-Golgi network"
}